{
  "gene": "UniProtKB:Q5HYJ1",
  "gene_name": "Trans-2,3-enoyl-CoA reductase-like",
  "gene_symbol": "TECRL",
  "term_id": "GO:0005783",
  "term_label": "endoplasmic reticulum"
}